heparan sulfate proteoglycan catabolic process [GO:0030200] (biological process) Relationships: is a type of proteoglycan catabolic process [GO:0030167]; is a type of heparan sulfate proteoglycan metabolic process [GO:0030201] References: PMID:35536982 Definition: The chemical reactions and pathways resulting in the breakdown of heparan sulfate proteoglycans, which consist of a core protein linked to a heparan sulfate glycosaminoglycan. The heparan sulfate chain is composed of the repeating disaccharide unit beta-(1,4)-N-acetyl-D-glucosamine-alpha-(1,4)-hexuronic acid, the former being either sulfated or deacetylated on its amino group as well as sulfated on one of its hydroxyl groups, and the latter being a mixture of sulfated and nonsulfated D-glucuronic and L-iduronic acids. Also known as: heparan sulfate proteoglycan breakdown, heparan sulfate proteoglycan catabolism, heparan sulfate proteoglycan degradation, heparan sulphate proteoglycan catabolic process, heparan sulphate proteoglycan catabolism, heparin proteoglycan catabolic process